{
  "gene": "UniProtKB:Q14738",
  "term_label": "protein phosphatase type 2A complex",
  "gene_name": "Serine_threonine-protein phosphatase 2A 56 kDa regulatory subunit delta isoform",
  "gene_symbol": "PPP2R5D",
  "term_id": "GO:0000159"
}